{
  "term_id": "UNKNOWN:0001",
  "gene_name": "Uncharacterized protein C1orf127",
  "gene_symbol": "C1orf127",
  "term_label": "Unknown molecular function",
  "gene": "UniProtKB:Q8N9H9"
}